{
  "gene_symbol": "IQCD",
  "gene": "UniProtKB:Q96DY2",
  "term_label": "Unknown biological process",
  "term_id": "UNKNOWN:0002",
  "gene_name": "Dynein regulatory complex protein 10"
}